alpha2-beta1 integrin-alpha3(VI) complex [GO:0070466] (cellular component) Definition: A protein complex that consists of an alpha2-beta1 integrin complex bound to a type VI collagen triple helix containing an alpha3(VI) chain. References: PMID:8387021 Relationships: is a type of plasma membrane protein complex [GO:0098797] Also known as: ITGA2-ITGB1-COL6A3 complex